plastid envelope [GO:0009526] (cellular component) Relationships: is a type of organelle envelope [GO:0031967]; is part of plastid [GO:0009536] Sources: GOC:jy Subtypes: GO:0009941, chromoplast envelope [GO:0031898], amyloplast envelope [GO:0033096], cyanelle envelope [GO:0033112], GO:0034425 Definition: The double lipid bilayer enclosing a plastid and separating its contents from the rest of the cytoplasm; includes the intermembrane space.